{
  "term_label": "syntaxin-3 binding",
  "gene_name": "Syntaxin-binding protein 2",
  "gene_symbol": "STXBP2",
  "term_id": "GO:0030348",
  "gene": "UniProtKB:Q15833"
}